viral budding from plasma membrane [GO:0046761] (biological process) Definition: A viral budding that starts with formation of a curvature in the host plasma membrane around which the virion particle assembles. References: PMID:9394621 Sources: GOC:bf, ISBN:0072370319, VZ:1947 Relationships: is a type of non-lytic viral release [GO:0046753]; is_a viral budding [GO:0046755] Also known as: plasma membrane viral budding, virus budding from plasma membrane, virus budding from plasma membrane by viral capsid envelopment, plasma membrane viral budding during viral capsid envelopment, viral budding from plasma membrane by viral capsid envelopment, viral budding from plasma membrane during viral capsid envelopment, virus budding from plasma membrane during viral capsid envelopment